cotyledon boundary formation [GO:0090451] (biological process) Definition: The process in which boundaries between a cotyledon and the surrounding tissue are established and maintained. Sources: GOC:tb Relationships: is a type of formation of plant organ boundary [GO:0090691]